{
  "term_label": "regulation of transcription by RNA polymerase II",
  "gene_name": "Neurotrophin receptor-interacting factor homolog",
  "term_id": "GO:0006357",
  "gene": "UniProtKB:Q96GC6",
  "gene_symbol": "ZNF274"
}